pyridoxamine phosphate oxidase activity [GO:0004733] (molecular function) References: PMID:11786019 Relationships: is a type of oxidoreductase activity, acting on the CH-NH2 group of donors, oxygen as acceptor [GO:0016641]; is part of GO:0042823 Definition: Catalysis of the reaction: pyridoxamine 5'-phosphate + H2O + O2 = pyridoxal 5'-phosphate + NH4+ + hydrogen peroxide. This activity can also oxidize pyridoxine 5'-phosphate to pyridoxal 5'-phosphate + hydrogen peroxide. Also known as: PMP oxidase activity, pyridoxal 5'-phosphate synthase activity, pyridoxamine 5'-phosphate oxidase activity, pyridoxamine-5'-phosphate:oxygen oxidoreductase (deaminating), pyridoxamine-phosphate oxidase activity, pyridoxaminephosphate oxidase deaminating, pyridoxine (pyridoxamine) 5'-phosphate oxidase activity, pyridoxine (pyridoxamine)phosphate oxidase activity